{
  "term_id": "UNKNOWN:0001",
  "term_label": "Unknown molecular function",
  "gene_symbol": "BLACE",
  "gene": "UniProtKB:A4D250",
  "gene_name": "B-cell acute lymphoblastic leukemia-expressed protein"
}